{
  "gene_name": "Low-density lipoprotein receptor-related protein 2",
  "term_id": "GO:0016324",
  "term_label": "apical plasma membrane",
  "gene": "UniProtKB:P98164",
  "gene_symbol": "LRP2"
}